{
  "gene": "UniProtKB:Q6ZS11",
  "term_label": "endocytic vesicle",
  "term_id": "GO:0030139",
  "gene_symbol": "RINL",
  "gene_name": "Ras and Rab interactor-like protein"
}